4-nitrophenol catabolic process [GO:0046196] (biological process) Relationships: is_a GO:0018960; is a type of GO:0019336; is a type of xenobiotic catabolic process [GO:0042178] Definition: The chemical reactions and pathways resulting in the breakdown of 4-nitrophenol, a nitroaromatic compound which is used in the production of dyes, leather treatment agents, fungicides and as an intermediate in the production of the insecticide parathion. Also known as: 4-nitrophenol breakdown, 4-nitrophenol catabolism, 4-nitrophenol degradation Sources: GOC:ai